{
  "gene_name": "Biorientation of chromosomes in cell division protein 1",
  "gene": "UniProtKB:Q96IK1",
  "term_id": "UNKNOWN:0001",
  "gene_symbol": "BOD1",
  "term_label": "Unknown molecular function"
}